{
  "term_label": "mitochondrion",
  "gene": "UniProtKB:Q8N465",
  "gene_symbol": "D2HGDH",
  "term_id": "GO:0005739",
  "gene_name": "D-2-hydroxyglutarate dehydrogenase, mitochondrial"
}